dATP biosynthetic process from ADP [GO:0006176] (BP) Relationships: is a type of dATP biosynthetic process [GO:0006175]; is_a ADP metabolic process [GO:0046031] Also known as: dATP anabolism from ADP, dATP formation from ADP, dATP synthesis from ADP Definition: The chemical reactions and pathways resulting in the formation of dATP, deoxyadenosine triphosphate (2'-deoxyadenosine 5'-triphosphate) from other compounds, including ADP, adenosine diphosphate. Sources: ISBN:0198506732